sulfate:bicarbonate antiporter activity [GO:0015383] (molecular function) Sources: TC:2.A.53.2.2 Definition: Enables the transfer of a solute or solutes from one side of a membrane to the other according to the reaction: sulfate(out) + bicarbonate(in) = sulfate(in) + bicarbonate(out). Also known as: sulfate:hydrogencarbonate antiporter activity, sulphate:bicarbonate antiporter activity Relationships: is a type of solute:inorganic anion antiporter activity [GO:0005452]; is a type of secondary active sulfate transmembrane transporter activity [GO:0008271]; is a type of bicarbonate transmembrane transporter activity [GO:0015106]